{
  "gene": "UniProtKB:Q9HD26",
  "gene_symbol": "GOPC",
  "term_label": "transmembrane transporter binding",
  "gene_name": "Golgi-associated PDZ and coiled-coil motif-containing protein",
  "term_id": "GO:0044325"
}